{
  "term_label": "inflammatory response",
  "gene_symbol": "TAC1",
  "term_id": "GO:0006954",
  "gene_name": "Protachykinin-1",
  "gene": "UniProtKB:P20366"
}